positive regulation of aplanospore formation [GO:0075291] (biological process) Sources: GOC:pamgo_curators Relationships: is a type of positive regulation of sporangiospore formation [GO:0075287]; is a type of regulation of aplanospore formation [GO:0075290]; positively regulates aplanospore formation [GO:0075289] Definition: Any process that activates, maintains or increases the frequency, rate or extent of aplanospore formation, a process in which a nonmotile, asexual spore is formed within a cell in certain algae and fungi (commonly in the Phycomycetes), the wall of aplanospore is distinct from that of the parent cell.